CRISPR-cas system [GO:0099048] (biological process) References: PMID:23495939, PMID:27302758, PMID:29440578 Relationships: is a type of clearance of foreign intracellular nucleic acids [GO:0099046] Definition: A defense response of that serves to clear host cells of foreign DNA and RNA. It has three distinct stage: acquisition of foreign DNA by integration into CRISPR loci in the host chromosome, CRISPR RNA (crRNA) biogenesis, and target interference. CRISPR stands for Clustered Regularly Interspaced Short Palindromic Repeat, which describes the nature of the loci.